positive regulation of tensidol B biosynthetic process [GO:1900712] (biological process) Also known as: activation of tensidol B anabolism, activation of tensidol B biosynthesis, activation of tensidol B formation, activation of tensidol B synthesis, positive regulation of tensidol B anabolism, positive regulation of tensidol B biosynthesis, positive regulation of tensidol B formation, positive regulation of tensidol B synthesis, up regulation of tensidol B anabolism, up regulation of tensidol B biosynthesis, up regulation of tensidol B biosynthetic process, up regulation of tensidol B formation, up regulation of tensidol B synthesis, up-regulation of tensidol B anabolism, up-regulation of tensidol B biosynthesis, up-regulation of tensidol B biosynthetic process, up-regulation of tensidol B formation, up-regulation of tensidol B synthesis, upregulation of tensidol B anabolism, upregulation of tensidol B biosynthesis, upregulation of tensidol B biosynthetic process, upregulation of tensidol B formation, upregulation of tensidol B synthesis, activation of tensidol B biosynthetic process Definition: Any process that activates or increases the frequency, rate or extent of tensidol B biosynthetic process. Sources: GOC:TermGenie, GOC:di Relationships: is a type of positive regulation of amide metabolic process [GO:0034250]; is a type of positive regulation of small molecule metabolic process [GO:0062013]; is_a positive regulation of secondary metabolite biosynthetic process [GO:1900378]; is a type of regulation of tensidol B biosynthetic process [GO:1900710]; positively regulates tensidol B biosynthetic process [GO:1900608]